arabinose biosynthetic process [GO:0019567] (biological process) Sources: GOC:ai Relationships: is a type of pentose biosynthetic process [GO:0019322]; is a type of GO:0019566 Subtypes: L-arabinose biosynthetic process [GO:0033357] Definition: The chemical reactions and pathways resulting in the formation of arabinose, arabino-pentose. Also known as: arabinose anabolism, arabinose biosynthesis, arabinose formation, arabinose synthesis